{
  "term_id": "GO:0045202",
  "gene": "UniProtKB:P22303",
  "gene_symbol": "ACHE",
  "term_label": "synapse",
  "gene_name": "Acetylcholinesterase"
}